positive regulation of starch utilization system complex assembly [GO:1900514] (biological process) Relationships: is a type of positive regulation of protein-containing complex assembly [GO:0031334]; is a type of regulation of starch utilization system complex assembly [GO:1900512]; positively regulates starch utilization system complex assembly [GO:0044574] Sources: GOC:TermGenie, GOC:mengo_curators Also known as: activation of SUS complex assembly, activation of assembly of starch utilization system complex, positive regulation of SUS complex assembly, positive regulation of assembly of starch utilization system complex, up regulation of SUS complex assembly, up regulation of assembly of starch utilization system complex, up regulation of starch utilization system complex assembly, up-regulation of SUS complex assembly, up-regulation of assembly of starch utilization system complex, up-regulation of starch utilization system complex assembly, upregulation of SUS complex assembly, upregulation of assembly of starch utilization system complex, upregulation of starch utilization system complex assembly, activation of starch utilization system complex assembly Definition: Any process that activates or increases the frequency, rate or extent of starch utilization system complex assembly.